{
  "gene_name": "Suppressor of cytokine signaling 6",
  "gene": "UniProtKB:O14544",
  "term_label": "signaling adaptor activity",
  "gene_symbol": "SOCS6",
  "term_id": "GO:0035591"
}